{
  "gene_symbol": "CHMP4C",
  "term_label": "Unknown molecular function",
  "term_id": "UNKNOWN:0001",
  "gene_name": "Charged multivesicular body protein 4c",
  "gene": "UniProtKB:Q96CF2"
}